{
  "gene": "UniProtKB:Q56P42",
  "term_label": "Unknown molecular function",
  "gene_name": "Pyrin domain-containing protein 2",
  "gene_symbol": "PYDC2",
  "term_id": "UNKNOWN:0001"
}